{
  "gene_symbol": "ESX1",
  "term_id": "GO:0006357",
  "gene": "UniProtKB:Q8N693",
  "term_label": "regulation of transcription by RNA polymerase II",
  "gene_name": "Homeobox protein ESX1"
}